{
  "gene": "UniProtKB:P36544",
  "gene_symbol": "CHRNA7",
  "term_id": "GO:0005886",
  "term_label": "plasma membrane",
  "gene_name": "Neuronal acetylcholine receptor subunit alpha-7"
}